{
  "gene_name": "HLA class I histocompatibility antigen, alpha chain E",
  "gene_symbol": "HLA-E",
  "gene": "UniProtKB:P13747",
  "term_id": "GO:0002476",
  "term_label": "antigen processing and presentation of endogenous peptide antigen via MHC class Ib"
}